{
  "gene_symbol": "XIRP1",
  "gene_name": "Xin actin-binding repeat-containing protein 1",
  "gene": "UniProtKB:Q702N8",
  "term_label": "actin filament organization",
  "term_id": "GO:0007015"
}